positive regulation of galactomannan catabolic process [GO:2000993] (biological process) Definition: Any process that activates or increases the frequency, rate or extent of galactomannan catabolic process. Relationships: is a type of positive regulation of catabolic process [GO:0009896]; is a type of positive regulation of macromolecule metabolic process [GO:0010604]; is a type of positive regulation of carbohydrate metabolic process [GO:0045913]; is a type of regulation of galactomannan catabolic process [GO:2000991]; positively regulates galactomannan catabolic process [GO:0051682] Sources: GOC:mengo_curators